{
  "term_label": "regulation of cell migration",
  "gene": "UniProtKB:O60486",
  "gene_symbol": "PLXNC1",
  "gene_name": "Plexin-C1",
  "term_id": "GO:0030334"
}